{
  "gene_name": "Nuclear pore complex protein Nup107",
  "gene": "UniProtKB:P57740",
  "gene_symbol": "NUP107",
  "term_id": "GO:0006406",
  "term_label": "mRNA export from nucleus"
}